{
  "gene_symbol": "STMN4",
  "term_label": "neuron projection",
  "gene": "UniProtKB:Q9H169",
  "term_id": "GO:0043005",
  "gene_name": "Stathmin-4"
}